{
  "gene_symbol": "RPS21",
  "term_label": "endonucleolytic cleavage in ITS1 to separate SSU-rRNA from 5.8S rRNA and LSU-rRNA from tricistronic rRNA transcript (SSU-rRNA, 5.8S rRNA, LSU-rRNA)",
  "gene": "UniProtKB:P63220",
  "gene_name": "Small ribosomal subunit protein eS21",
  "term_id": "GO:0000447"
}